regulation of granulocyte colony-stimulating factor production [GO:0071655] (biological process) Relationships: is a type of regulation of macrophage colony-stimulating factor production [GO:1901256]; regulates granulocyte colony-stimulating factor production [GO:0071611] Subtypes: GO:0071656, positive regulation of granulocyte colony-stimulating factor production [GO:0071657] Sources: GOC:mah Also known as: regulation of CSF3 production, regulation of G-CSF production, regulation of colony stimulating factor 3 (granulocyte) production, regulation of filgrastim production, regulation of granulocyte colony stimulating factor production, regulation of lenograstim production, regulation of pluripoietin production Definition: Any process that modulates the frequency, rate, or extent of production of granulocyte colony-stimulating factor.